{
  "term_id": "GO:0016020",
  "gene_name": "Mitochondrial carrier homolog 1",
  "gene_symbol": "MTCH1",
  "term_label": "membrane",
  "gene": "UniProtKB:Q9NZJ7"
}